cytoplasmic microtubule depolymerization [GO:0010938] (biological process) Definition: The removal of tubulin heterodimers from one or both ends of a cytoplasmic microtubule. Sources: GOC:dph, GOC:tb Relationships: is a type of GO:0007019; is a type of cytoplasmic microtubule organization [GO:0031122]; occurs in cytoplasm [GO:0005737] Subtypes: axonemal microtubule depolymerization [GO:0060404] Regulation: regulated by regulation of cytoplasmic microtubule depolymerization [GO:0010937]